{
  "term_id": "GO:0051015",
  "gene_symbol": "ABITRAM",
  "gene": "UniProtKB:Q9NX38",
  "term_label": "actin filament binding",
  "gene_name": "Protein Abitram"
}